{
  "term_id": "UNKNOWN:0002",
  "term_label": "Unknown biological process",
  "gene": "UniProtKB:P59861",
  "gene_symbol": "DEFB131A",
  "gene_name": "Beta-defensin 131A"
}